{
  "term_id": "GO:0045202",
  "term_label": "synapse",
  "gene_name": "Muscarinic acetylcholine receptor M2",
  "gene": "UniProtKB:P08172",
  "gene_symbol": "CHRM2"
}